{
  "gene_name": "T-complex protein 11 X-linked protein 1",
  "gene": "UniProtKB:B4DZS4",
  "term_label": "acrosomal vesicle",
  "gene_symbol": "TCP11X1",
  "term_id": "GO:0001669"
}